{
  "term_label": "regulation of epidermal growth factor receptor signaling pathway",
  "term_id": "GO:0042058",
  "gene_name": "Inactive rhomboid protein 1",
  "gene": "UniProtKB:Q96CC6",
  "gene_symbol": "RHBDF1"
}